{
  "gene_name": "Exostosin-like 3",
  "term_id": "GO:0005794",
  "gene_symbol": "EXTL3",
  "gene": "UniProtKB:O43909",
  "term_label": "Golgi apparatus"
}